L-phenylalanine import across plasma membrane [GO:0140925] (biological process) Definition: The directed movement of L-phenylalanine from outside of a cell, across the plasma membrane and into the cytosol. References: PMID:11069779 Relationships: is a type of organic cation transport [GO:0015695]; is a type of aromatic amino acid transport [GO:0015801]; is a type of phenylalanine transport [GO:0015823]; is a type of GO:0089718; is a type of L-alpha-amino acid transmembrane transport [GO:1902475]